{
  "gene": "UniProtKB:O95841",
  "gene_symbol": "ANGPTL1",
  "gene_name": "Angiopoietin-related protein 1",
  "term_id": "GO:0007169",
  "term_label": "cell surface receptor protein tyrosine kinase signaling pathway"
}